{
  "gene_symbol": "KRBA2",
  "term_label": "Unknown molecular function",
  "term_id": "UNKNOWN:0001",
  "gene": "UniProtKB:Q6ZNG9",
  "gene_name": "KRAB-A domain-containing protein 2"
}